{
  "gene": "UniProtKB:Q5T5C0",
  "term_id": "GO:0006887",
  "term_label": "exocytosis",
  "gene_symbol": "STXBP5",
  "gene_name": "Syntaxin-binding protein 5"
}